{
  "gene_name": "Dimethyladenosine transferase 2, mitochondrial",
  "term_id": "GO:0031167",
  "term_label": "rRNA methylation",
  "gene": "UniProtKB:Q9H5Q4",
  "gene_symbol": "TFB2M"
}